{
  "term_label": "junctional membrane complex",
  "gene_symbol": "JPH4",
  "gene": "UniProtKB:Q96JJ6",
  "term_id": "GO:0030314",
  "gene_name": "Junctophilin-4"
}